positive regulation of cell adhesion involved in single-species biofilm formation [GO:1900189] (biological process) Relationships: is a type of positive regulation of cell-substrate adhesion [GO:0010811]; is a type of regulation of cell adhesion involved in single-species biofilm formation [GO:1900187]; RO_0002213 cell adhesion involved in single-species biofilm formation [GO:0043709] Definition: Any process that activates or increases the frequency, rate or extent of cell adhesion involved in single-species biofilm formation. Also known as: up regulation of cell adhesion involved in single-species biofilm formation, up-regulation of cell adhesion involved in single-species biofilm formation, upregulation of cell adhesion involved in single-species biofilm formation, activation of cell adhesion involved in single-species biofilm formation, activation of cell adhesion during single-species biofilm formation, positive regulation of cell adhesion during single-species biofilm formation, up regulation of cell adhesion during single-species biofilm formation, up-regulation of cell adhesion during single-species biofilm formation, upregulation of cell adhesion during single-species biofilm formation Sources: GOC:TermGenie, GOC:di